{
  "gene_symbol": "RBP2",
  "term_id": "GO:0005829",
  "term_label": "cytosol",
  "gene_name": "Retinol-binding protein 2",
  "gene": "UniProtKB:P50120"
}